{
  "gene_name": "Mesogenin-1",
  "term_label": "nucleus",
  "gene_symbol": "MSGN1",
  "term_id": "GO:0005634",
  "gene": "UniProtKB:A6NI15"
}